adrenomedullin binding [GO:1990409] (molecular function) Definition: Binding to adrenomedullin (AM). Also known as: AM binding References: PMID:10882736 Sources: GOC:bhm Note: An example of a protein that could be annotated to this term is CALCRL in human (Q16602) in PMID:10882736. Relationships: is_a calcitonin family binding [GO:0097644]